rod photoreceptor outer segment [GO:0120200] (cellular component) Relationships: is_a photoreceptor outer segment [GO:0001750] Definition: The outer segment of a vertebrate rod photoreceptor that contains sealed membrane discs that are not connected to the ciliary membrane and containing rhodopsin photoreceptor proteins. References: PMID:19501669, PMID:26574505, PMID:6771304 Sources: GOC:krc, GOC:pde